{
  "gene_name": "CLK4-associating serine_arginine rich protein",
  "gene": "UniProtKB:Q8N2M8",
  "term_label": "Unknown biological process",
  "term_id": "UNKNOWN:0002",
  "gene_symbol": "CLASRP"
}